{
  "gene_name": "Angiogenic factor with G patch and FHA domains 1",
  "term_id": "UNKNOWN:0003",
  "term_label": "Unknown cellular component",
  "gene_symbol": "AGGF1",
  "gene": "UniProtKB:Q8N302"
}